{
  "gene_name": "Semaphorin-3B",
  "term_label": "plasma membrane",
  "gene": "UniProtKB:Q13214",
  "gene_symbol": "SEMA3B",
  "term_id": "GO:0005886"
}